{
  "gene": "UniProtKB:P00505",
  "term_label": "L-aspartate catabolic process",
  "gene_symbol": "GOT2",
  "gene_name": "Aspartate aminotransferase, mitochondrial",
  "term_id": "GO:0006533"
}